histone H4R3 demethylase activity [GO:0033749] (molecular function) Definition: Catalysis of the removal of the methyl group from a modified arginine residue at position 3 of the histone H4 protein. This is a dioxygenase reaction that is dependent on Fe(II) and 2-oxoglutarate. Relationships: is a type of 2-oxoglutarate-dependent dioxygenase activity [GO:0016706]; is a type of histone H4 demethylase activity [GO:0141058] Also known as: histone H4-methyl-arginine-3 demethylase activity, histone H4R3me demethylase activity, histone demethylase activity (H4-R3 specific) References: PMID:17947579 Note: Note that the residue position corresponds to the canonical human H4 histone (UniProtKB:P02309); this residue is conserved across all eukaryotes. Note that the initiation methionine is cleaved, so the first residue is S1.